{
  "gene_symbol": "MNX1",
  "gene_name": "Motor neuron and pancreas homeobox protein 1",
  "term_label": "nucleus",
  "gene": "UniProtKB:P50219",
  "term_id": "GO:0005634"
}